growth plate cartilage chondrocyte differentiation [GO:0003418] (biological process) Relationships: is a type of chondrocyte differentiation involved in endochondral bone morphogenesis [GO:0003413]; is part of GO:0003417 Regulation: regulated by regulation of growth plate cartilage chondrocyte differentiation [GO:1902733] Sources: GOC:ascb_2009, GOC:dph, GOC:tb Definition: The process in which a chondroblast acquires specialized structural and/or functional features of a chondrocyte that will contribute to the growth of a bone. A chondrocyte is a polymorphic cell that forms cartilage.